IAA-amino acid conjugate hydrolase activity [GO:0010178] (molecular function) Relationships: is a type of hydrolase activity, acting on carbon-nitrogen (but not peptide) bonds [GO:0016810] Definition: Catalysis of the cleavage of the amide bond between IAA (auxin) and the conjugated amino acid. Sources: GOC:tb Subtypes: IAA-Ala conjugate hydrolase activity [GO:0010179], GO:0010210, GO:0010211